negative regulation of the force of heart contraction [GO:0098736] (biological process) Relationships: is a type of regulation of the force of heart contraction [GO:0002026] References: PMID:17242280 Sources: GOC:BHF, GOC:dos, GOC:mtg_cardiac_conduct_nov11, GOC:rl Definition: Any process that decreases the force of heart muscle contraction.